positive regulation of hair follicle cell proliferation [GO:0071338] (biological process) Definition: Any process that activates or increases the rate or extent of hair follicle cell proliferation. Sources: GOC:mah Relationships: is a type of GO:0008284; is a type of regulation of hair follicle cell proliferation [GO:0071336]; positively regulates hair follicle cell proliferation [GO:0071335] Also known as: up regulation of hair follicle cell proliferation, up-regulation of hair follicle cell proliferation, upregulation of hair follicle cell proliferation, activation of hair follicle cell proliferation, stimulation of hair follicle cell proliferation